protein-lipid complex assembly [GO:0065005] (biological process) Definition: The aggregation, arrangement and bonding together of proteins and lipids to form a protein-lipid complex. Sources: GOC:jl Relationships: is a type of protein-containing complex assembly [GO:0065003]; is a type of GO:0071825 Subtypes: GO:0002493, plasma lipoprotein particle assembly [GO:0034377], lipid tube assembly [GO:0060988]